{
  "gene_name": "Calcium homeostasis modulator protein 5",
  "gene": "UniProtKB:Q8N5C1",
  "term_label": "Unknown biological process",
  "gene_symbol": "CALHM5",
  "term_id": "UNKNOWN:0002"
}